{
  "term_label": "DNA replication",
  "term_id": "GO:0006260",
  "gene_name": "Single-stranded DNA-binding protein, mitochondrial",
  "gene_symbol": "SSBP1",
  "gene": "UniProtKB:Q04837"
}